{
  "gene_symbol": "CXCL13",
  "term_label": "neutrophil chemotaxis",
  "gene_name": "C-X-C motif chemokine 13",
  "gene": "UniProtKB:O43927",
  "term_id": "GO:0030593"
}